renal interstitial fibroblast fate commitment [GO:0072153] (biological process) Also known as: kidney interstitial cell fate commitment Definition: The process in which the developmental fate of a cell becomes restricted such that it will develop into a renal fibroblast. Sources: GOC:mtg_kidney_jan10 Subtypes: mesonephric interstitial fibroblast fate commitment [GO:0061268], GO:0072260 Relationships: is a type of GO:0045165; is part of kidney interstitial fibroblast differentiation [GO:0072071]